{
  "term_id": "UNKNOWN:0001",
  "term_label": "Unknown molecular function",
  "gene": "UniProtKB:Q15238",
  "gene_symbol": "PSG5",
  "gene_name": "Pregnancy-specific beta-1-glycoprotein 5"
}